negative regulation of adenosine transport [GO:0032250] (biological process) Also known as: down regulation of adenosine transport, down-regulation of adenosine transport, downregulation of adenosine transport, inhibition of adenosine transport Definition: Any process that stops, prevents, or reduces the frequency, rate or extent of the directed movement of adenosine into, out of or within a cell, or between cells, by means of some agent such as a transporter or pore. Relationships: is a type of negative regulation of purine nucleoside transport [GO:0032247]; is a type of regulation of adenosine transport [GO:0032249]; negatively regulates GO:0032238 Sources: GOC:mah